{
  "term_label": "Unknown biological process",
  "gene_symbol": "TP53AIP1",
  "term_id": "UNKNOWN:0002",
  "gene_name": "p53-regulated apoptosis-inducing protein 1",
  "gene": "UniProtKB:Q9HCN2"
}